{
  "gene_symbol": "TPRX2",
  "term_label": "RNA polymerase II cis-regulatory region sequence-specific DNA binding",
  "gene_name": "Tetrapeptide repeat homeobox protein 2",
  "term_id": "GO:0000978",
  "gene": "UniProtKB:P0DV77"
}